positive regulation of mitochondrial outer membrane permeabilization involved in apoptotic signaling pathway [GO:1901030] (biological process) Sources: GOC:BHF, GOC:TermGenie, GOC:mtg_apoptosis Definition: Any process that activates or increases the frequency, rate or extent of mitochondrial outer membrane permeabilization involved in apoptotic signaling pathway. Note: Caspase 8 may be annotated to this term when it is shown to stimulate MOMP by cleaving the BH3-only protein BID. Also known as: positive regulation of mitochondrial outer membrane permeabilization, positive regulation of MOMP, up regulation of MOMP, up regulation of mitochondrial outer membrane permeabilization, up-regulation of MOMP, up-regulation of mitochondrial outer membrane permeabilization, upregulation of MOMP, upregulation of mitochondrial outer membrane permeabilization, activation of MOMP, activation of mitochondrial outer membrane permeabilization Relationships: is a type of positive regulation of organelle organization [GO:0010638]; is a type of positive regulation of mitochondrial membrane permeability [GO:0035794]; is a type of positive regulation of transport [GO:0051050]; is a type of regulation of mitochondrial outer membrane permeabilization involved in apoptotic signaling pathway [GO:1901028]; positively regulates GO:0097345